regulation of vasoconstriction by neuronal norepinephrine [GO:0003118] (biological process) Also known as: regulation of vasoconstriction by neuronal noradrenaline Sources: GOC:mtg_cardio Definition: Any process that modulates the frequency, rate or extent of reductions in the diameter of blood vessels as a result of norepinephrine released by nerve endings. Relationships: is a type of regulation of vasoconstriction by norepinephrine [GO:0003116]